{
  "gene_name": "Zinc finger protein 101",
  "term_label": "nucleus",
  "gene_symbol": "ZNF101",
  "gene": "UniProtKB:Q8IZC7",
  "term_id": "GO:0005634"
}